vanadium ion binding [GO:0051212] (molecular function) Definition: Binding to a vanadium ion (V). Sources: GOC:ai Relationships: is a type of transition metal ion binding [GO:0046914] Also known as: V ion binding